constitutive heterochromatin formation [GO:0140719] (biological process) Note: Note that constitutive heterochromatin usually cannot be reprogrammed to a transcriptionally-competent state, as opposed to facultative heterochromatin, which can be reprogrammed. Note also that constitutive usually involves DNA methylation, while facultative heterochromatin formation does not. Also known as: constitutive heterochromatin assembly Relationships: is a type of heterochromatin formation [GO:0031507] Subtypes: GO:0006346, silent mating-type cassette heterochromatin formation [GO:0030466], pericentric heterochromatin formation [GO:0031508], GO:0031509, transposable element silencing by heterochromatin formation [GO:0141005] References: PMID:17936700 Definition: The compaction of chromatin into heterochromatin, a conformation that is refractory to transcription. Constitutive heterochromatin cannot be converted back to euchromatin, the transcriptionally-active conformation. In metazoa, this involves the methylation of histone H3K9.